tripartite ATP-independent periplasmic transporter complex [GO:0031317] (cellular component) Also known as: TRAP transporter complex, TRAP-T transporter complex Sources: GOC:mlg Definition: A complex consisting of two membrane proteins and one extracytoplasmic solute receptor. Such transporters transport a variety of substrates without direct ATP power, instead using energy from ion gradients. Relationships: is a type of transporter complex [GO:1990351]